negative regulation of L-ascorbic acid biosynthetic process [GO:2000083] (biological process) Definition: Any process that stops, prevents, or reduces the frequency, rate or extent of L-ascorbic acid biosynthetic process. References: PMID:19395407 Relationships: is a type of negative regulation of biosynthetic process [GO:0009890]; is a type of negative regulation of carbohydrate metabolic process [GO:0045912]; is a type of GO:0046137; is a type of regulation of L-ascorbic acid biosynthetic process [GO:2000082]; RO_0002212 L-ascorbic acid biosynthetic process [GO:0019853] Also known as: negative regulation of L-ascorbic acid anabolism, negative regulation of L-ascorbic acid biosynthesis, negative regulation of L-ascorbic acid formation, negative regulation of L-ascorbic acid synthesis, negative regulation of ascorbate biosynthesis, negative regulation of ascorbate biosynthetic process, negative regulation of vitamin C biosynthesis, negative regulation of vitamin C biosynthetic process